negative regulation of myotube cell migration [GO:0110125] (BP) Relationships: is a type of negative regulation of cell migration [GO:0030336]; is a type of regulation of myotube cell migration [GO:0110123]; negatively regulates myotube cell migration [GO:0110122] Definition: Any process that stops, prevents, or reduces the frequency, rate or extent of myotube cell migration. References: PMID:29122742 Sources: GOC:ha